zeatin reductase activity [GO:0050472] (molecular function) Sources: EC:1.3.1.69, RHEA:12757 Relationships: is a type of oxidoreductase activity, acting on the CH-CH group of donors, NAD or NADP as acceptor [GO:0016628] Also known as: dihydrozeatin:NADP+ oxidoreductase activity Definition: Catalysis of the reaction: dihydrozeatin + NADP+ = H+ + NADPH + zeatin.